{
  "gene_symbol": "APH1B",
  "gene_name": "Gamma-secretase subunit APH-1B",
  "term_id": "GO:0007219",
  "gene": "UniProtKB:Q8WW43",
  "term_label": "Notch signaling pathway"
}